{
  "term_label": "axon",
  "term_id": "GO:0030424",
  "gene": "UniProtKB:Q9UHY8",
  "gene_symbol": "FEZ2",
  "gene_name": "Fasciculation and elongation protein zeta-2"
}